spine apparatus [GO:0097444] (cellular component) Also known as: dense material Definition: A specialization of the endomembrane system found in some classes of dendritic spines consisting of two or more closely apposed lamellae with interspersed electron dense material. The endomembrane component is continuous with the smooth endoplasmic reticulum. Relationships: is a type of membrane-bounded organelle [GO:0043227]; is part of endomembrane system [GO:0012505]; is part of dendritic spine [GO:0043197] References: PMID:20400711, PMID:8987748 Sources: NIF_Subcellular:sao725931194